{
  "gene_symbol": "RAB39A",
  "term_label": "vesicle-mediated transport",
  "gene_name": "Ras-related protein Rab-39A",
  "gene": "UniProtKB:Q14964",
  "term_id": "GO:0016192"
}